{
  "term_label": "regulation of mRNA splicing, via spliceosome",
  "gene": "UniProtKB:Q96PU8",
  "term_id": "GO:0048024",
  "gene_name": "KH domain-containing RNA-binding protein QKI",
  "gene_symbol": "QKI"
}